{
  "gene_name": "Probable cysteine--tRNA ligase, mitochondrial",
  "term_label": "cysteinyl-tRNA aminoacylation",
  "gene_symbol": "CARS2",
  "gene": "UniProtKB:Q9HA77",
  "term_id": "GO:0006423"
}